{
  "gene": "UniProtKB:Q8IV03",
  "gene_name": "Leucine rich adaptor protein 1-like",
  "gene_symbol": "LURAP1L",
  "term_label": "Unknown biological process",
  "term_id": "UNKNOWN:0002"
}